2-dehydro-3-deoxy-D-gluconate aldolase activity [GO:0061677] (molecular function) References: PMID:12824170 Sources: GOC:dph, RHEA:35583 Definition: Catalysis of the reaction: 2-dehydro-3-deoxy-D-gluconate = pyruvate + D-glyceraldehyde. Relationships: is a type of aldehyde-lyase activity [GO:0016832] Also known as: 2-keto-3-deoxygluconate aldolase activity, KDG aldolase activity